{
  "gene": "UniProtKB:Q9NXL2",
  "gene_symbol": "ARHGEF38",
  "term_id": "GO:0005085",
  "term_label": "guanyl-nucleotide exchange factor activity",
  "gene_name": "Rho guanine nucleotide exchange factor 38"
}